{
  "gene": "UniProtKB:A0A0U1RR37",
  "term_label": "Unknown biological process",
  "term_id": "UNKNOWN:0002",
  "gene_symbol": "C1orf232",
  "gene_name": "Uncharacterized protein C1orf232"
}